{
  "term_label": "microtubule binding",
  "gene": "UniProtKB:Q9Y4F4",
  "term_id": "GO:0008017",
  "gene_name": "TOG array regulator of axonemal microtubules protein 1",
  "gene_symbol": "TOGARAM1"
}